{
  "gene_name": "Integrin alpha-5",
  "gene": "UniProtKB:P08648",
  "term_label": "signaling receptor activity",
  "gene_symbol": "ITGA5",
  "term_id": "GO:0038023"
}